negative regulation of chlorophyll biosynthetic process [GO:1902325] (biological process) Also known as: down regulation of chlorophyll anabolism, down regulation of chlorophyll biosynthesis, down regulation of chlorophyll biosynthetic process, down regulation of chlorophyll formation, down regulation of chlorophyll synthesis, down-regulation of chlorophyll anabolism, down-regulation of chlorophyll biosynthesis, down-regulation of chlorophyll biosynthetic process, down-regulation of chlorophyll formation, down-regulation of chlorophyll synthesis, downregulation of chlorophyll anabolism, downregulation of chlorophyll biosynthesis, downregulation of chlorophyll biosynthetic process, downregulation of chlorophyll formation, downregulation of chlorophyll synthesis, negative regulation of chlorophyll anabolism, negative regulation of chlorophyll biosynthesis, negative regulation of chlorophyll formation, negative regulation of chlorophyll synthesis, inhibition of chlorophyll anabolism, inhibition of chlorophyll biosynthesis, inhibition of chlorophyll biosynthetic process, inhibition of chlorophyll formation, inhibition of chlorophyll synthesis Relationships: is a type of regulation of chlorophyll biosynthetic process [GO:0010380]; is a type of negative regulation of tetrapyrrole biosynthetic process [GO:1901464]; negatively regulates chlorophyll biosynthetic process [GO:0015995] References: PMID:23555952 Sources: GOC:TermGenie Definition: Any process that stops, prevents or reduces the frequency, rate or extent of chlorophyll biosynthetic process.